synaptotagmin-synaptobrevin 2-SNAP-25-syntaxin-1a-syntaxin-1b-Rab3a-complexin II complex [GO:0070355] (cellular component) Relationships: is a type of GO:0031201 Definition: A SNARE complex that contains synaptotagmin, synaptobrevin 2 (VAMP2), SNAP-25, syntaxin 1a, syntaxin1b, Rab3a, and complexin II (or orthologs thereof). Also known as: SNARE complex (STX1a, STX1b, SNAP25, RAB3a, SYT1, VAMP2, CPLX2), STX1a-STX1b-SNAP25-RAB3a-SYT1-VAMP2-CPLX2 complex References: PMID:7654227